{
  "gene_symbol": "STT3B",
  "gene": "UniProtKB:Q8TCJ2",
  "term_label": "protein N-linked glycosylation via asparagine",
  "term_id": "GO:0018279",
  "gene_name": "Dolichyl-diphosphooligosaccharide--protein glycosyltransferase subunit STT3B"
}